sucrose-phosphate synthase activity [GO:0046524] (molecular function) Definition: Catalysis of the reaction: UDP-glucose + D-fructose 6-phosphate = UDP + sucrose 6-phosphate. Sources: EC:2.4.1.14 Also known as: SPS, UDP-glucose-fructose-phosphate glucosyltransferase activity, UDP-glucose:D-fructose-6-phosphate 2-alpha-D-glucosyltransferase activity, UDPglucose-fructose-phosphate glucosyltransferase activity, UDPglucose:D-fructose-6-phosphate 2-alpha-D-glucosyltransferase activity, sucrose 6-phosphate synthase activity, sucrose phosphate synthetase activity, sucrose phosphate-uridine diphosphate glucosyltransferase activity, sucrosephosphate-UDP glucosyltransferase activity, uridine diphosphoglucose-fructose phosphate glucosyltransferase activity Relationships: is a type of GO:0035251